{
  "gene_symbol": "AKNA",
  "gene_name": "Microtubule organization protein AKNA",
  "gene": "UniProtKB:Q7Z591",
  "term_id": "UNKNOWN:0001",
  "term_label": "Unknown molecular function"
}